{
  "gene": "UniProtKB:Q99550",
  "term_label": "centriole",
  "gene_symbol": "MPHOSPH9",
  "gene_name": "M-phase phosphoprotein 9",
  "term_id": "GO:0005814"
}